mitochondrial unfolded protein response [GO:0034514] (biological process) Definition: The series of molecular signals generated as a consequence of the presence of unfolded proteins in the mitochondrial matrix; results in transcriptional upregulation of nuclear genes encoding mitochondrial stress proteins. References: PMID:17849004 Sources: GOC:mah Also known as: mtUPR Relationships: is a type of cellular response to unfolded protein [GO:0034620]